{
  "gene_symbol": "NANOS3",
  "gene_name": "Nanos homolog 3",
  "term_label": "perinuclear region of cytoplasm",
  "gene": "UniProtKB:P60323",
  "term_id": "GO:0048471"
}